alpha-glucoside:proton symporter activity [GO:0005352] (molecular function) Also known as: general alpha-glucoside transporter activity, alpha-glucoside:hydrogen symporter activity, general alpha-glucoside:hydrogen symporter activity, general alpha-glucoside:proton symporter activity Definition: Enables the transfer of a solute or solutes from one side of a membrane to the other according to the reaction: alpha-glucoside(out) + H+(out) = alpha-glucoside(in) + H+(in). Alpha-glucosides include trehalose, maltose, turanose, isomaltose, alpha-methylglucoside, maltotriose, palatinose, trehalose and melezitose. Relationships: is a type of alpha-glucoside transmembrane transporter activity [GO:0015151]; is a type of solute:proton symporter activity [GO:0015295] Sources: TC:2.A.1.1.11